{
  "gene": "UniProtKB:A0A1B0GTE1",
  "gene_name": "Contactin associated protein family member 3C (Fragment)",
  "term_label": "Unknown biological process",
  "gene_symbol": "CNTNAP3C",
  "term_id": "UNKNOWN:0002"
}